{
  "gene_symbol": "NR2E3",
  "term_id": "GO:0045944",
  "gene_name": "Photoreceptor-specific nuclear receptor",
  "gene": "UniProtKB:Q9Y5X4",
  "term_label": "positive regulation of transcription by RNA polymerase II"
}